{
  "gene_symbol": "FAM83D",
  "term_id": "GO:0097431",
  "term_label": "mitotic spindle pole",
  "gene": "UniProtKB:Q9H4H8",
  "gene_name": "Protein FAM83D"
}